{
  "term_id": "GO:0009897",
  "gene_name": "CD27 antigen",
  "term_label": "external side of plasma membrane",
  "gene_symbol": "CD27",
  "gene": "UniProtKB:P26842"
}